{
  "term_id": "GO:0003924",
  "gene": "UniProtKB:A4D1E9",
  "gene_name": "GTP-binding protein 10",
  "gene_symbol": "GTPBP10",
  "term_label": "GTPase activity"
}